{
  "gene_symbol": "TRIM3",
  "gene": "UniProtKB:O75382",
  "gene_name": "Tripartite motif-containing protein 3",
  "term_id": "GO:0000209",
  "term_label": "protein polyubiquitination"
}